{
  "gene": "UniProtKB:K7EIQ3",
  "term_label": "Unknown cellular component",
  "term_id": "UNKNOWN:0003",
  "gene_symbol": "ZNF561-AS1",
  "gene_name": "Uncharacterized protein ZNF561-AS1"
}